{
  "gene": "UniProtKB:O60292",
  "gene_symbol": "SIPA1L3",
  "gene_name": "Signal-induced proliferation-associated 1-like protein 3",
  "term_label": "plasma membrane",
  "term_id": "GO:0005886"
}